{
  "gene": "UniProtKB:Q9UGN5",
  "term_id": "GO:0005730",
  "term_label": "nucleolus",
  "gene_symbol": "PARP2",
  "gene_name": "Poly [ADP-ribose] polymerase 2"
}